{
  "gene_name": "Formin-binding protein 1",
  "gene_symbol": "FNBP1",
  "term_id": "UNKNOWN:0003",
  "term_label": "Unknown cellular component",
  "gene": "UniProtKB:Q96RU3"
}